{
  "term_id": "UNKNOWN:0001",
  "gene_name": "Putative uncharacterized protein DKFZp434L187",
  "gene_symbol": "Q9UFV3",
  "gene": "UniProtKB:Q9UFV3",
  "term_label": "Unknown molecular function"
}